{
  "gene_name": "Sodium_hydrogen exchanger 7",
  "term_id": "GO:0005886",
  "term_label": "plasma membrane",
  "gene": "UniProtKB:Q96T83",
  "gene_symbol": "SLC9A7"
}